{
  "term_id": "GO:0000122",
  "gene_symbol": "PLAGL1",
  "gene_name": "Zinc finger protein PLAGL1",
  "term_label": "negative regulation of transcription by RNA polymerase II",
  "gene": "UniProtKB:Q9UM63"
}